{
  "term_label": "ubiquitin-like ligase-substrate adaptor activity",
  "term_id": "GO:1990756",
  "gene": "UniProtKB:Q9NVR0",
  "gene_name": "Kelch-like protein 11",
  "gene_symbol": "KLHL11"
}